{
  "gene_name": "Syntaxin-1B",
  "gene_symbol": "STX1B",
  "term_id": "GO:0000149",
  "term_label": "SNARE binding",
  "gene": "UniProtKB:P61266"
}